{
  "gene_symbol": "ITGB7",
  "gene": "UniProtKB:P26010",
  "term_label": "cell-matrix adhesion",
  "gene_name": "Integrin beta-7",
  "term_id": "GO:0007160"
}